{
  "term_label": "sphingolipid biosynthetic process",
  "gene_name": "Elongation of very long chain fatty acids protein 1",
  "gene_symbol": "ELOVL1",
  "term_id": "GO:0030148",
  "gene": "UniProtKB:Q9BW60"
}